{
  "term_id": "GO:0072583",
  "gene_name": "Clathrin light chain A",
  "term_label": "clathrin-dependent endocytosis",
  "gene_symbol": "CLTA",
  "gene": "UniProtKB:P09496"
}